{
  "term_id": "UNKNOWN:0002",
  "gene": "UniProtKB:Q92623",
  "gene_symbol": "TTC9",
  "term_label": "Unknown biological process",
  "gene_name": "Tetratricopeptide repeat protein 9A"
}